{
  "gene": "UniProtKB:Q8IWR0",
  "gene_symbol": "ZC3H7A",
  "term_id": "GO:0035196",
  "term_label": "miRNA processing",
  "gene_name": "Zinc finger CCCH domain-containing protein 7A"
}